{
  "gene_name": "Activin receptor type-2B",
  "term_id": "GO:0048185",
  "gene_symbol": "ACVR2B",
  "term_label": "activin binding",
  "gene": "UniProtKB:Q13705"
}